{
  "gene": "UniProtKB:A6NKQ9",
  "gene_symbol": "CGB1",
  "term_id": "GO:0005615",
  "gene_name": "Choriogonadotropin subunit beta variant 1",
  "term_label": "extracellular space"
}